{
  "gene_symbol": "MECOM",
  "gene": "UniProtKB:Q03112",
  "term_label": "DNA-binding transcription activator activity, RNA polymerase II-specific",
  "term_id": "GO:0001228",
  "gene_name": "Histone-lysine N-methyltransferase MECOM"
}